{
  "gene_symbol": "CTSL",
  "gene_name": "Procathepsin L",
  "term_label": "proteolysis involved in protein catabolic process",
  "gene": "UniProtKB:P07711",
  "term_id": "GO:0051603"
}